tRNA binding [GO:0000049] (molecular function) Subtypes: GO:0030557, methionyl-initiator methionine tRNA binding [GO:1990856] Also known as: base pairing with tRNA Sources: GOC:ai Relationships: is a type of RNA binding [GO:0003723] Definition: Binding to a transfer RNA.